{
  "gene": "UniProtKB:Q05329",
  "gene_symbol": "GAD2",
  "term_label": "gamma-aminobutyric acid biosynthetic process",
  "gene_name": "Glutamate decarboxylase 2",
  "term_id": "GO:0009449"
}